{
  "term_label": "Ral protein signal transduction",
  "gene": "UniProtKB:Q9NYS0",
  "term_id": "GO:0032484",
  "gene_symbol": "NKIRAS1",
  "gene_name": "NF-kappa-B inhibitor-interacting Ras-like protein 1"
}